neurotransmitter loading into synaptic vesicle [GO:0098700] (biological process) Regulation: regulated by GO:0099162 Also known as: neurotransmitter import into synaptic vesicle, neurotransmitter uptake into synaptic vesicle, synaptic vesicle neurotransmitter loading Definition: The active transport of neurotransmitters into a synaptic vesicle. This import is fuelled by an electrochemical gradient across the vesicle membrane, established by the action of proton pumps. Relationships: is a type of neurotransmitter transport [GO:0006836]; is a type of establishment of localization in cell [GO:0051649]; is part of synaptic vesicle cycle [GO:0099504] References: PMID:10099709, PMID:15217342 Sources: GOC:PARL, GOC:bf, GOC:pad Subtypes: GO:0015842